{
  "gene_symbol": "NRAP",
  "gene_name": "Nebulin-related-anchoring protein",
  "term_label": "cardiac muscle thin filament assembly",
  "term_id": "GO:0071691",
  "gene": "UniProtKB:Q86VF7"
}